{
  "gene_name": "Lipopolysaccharide-binding protein",
  "gene_symbol": "LBP",
  "term_label": "innate immune response",
  "term_id": "GO:0045087",
  "gene": "UniProtKB:P18428"
}